{
  "term_label": "cytoplasm",
  "gene": "UniProtKB:Q14344",
  "gene_symbol": "GNA13",
  "term_id": "GO:0005737",
  "gene_name": "Guanine nucleotide-binding protein subunit alpha-13"
}